{
  "gene": "UniProtKB:Q5T2D3",
  "term_label": "Unknown cellular component",
  "term_id": "UNKNOWN:0003",
  "gene_name": "OTU domain-containing protein 3",
  "gene_symbol": "OTUD3"
}